{
  "term_label": "Unknown molecular function",
  "gene_symbol": "CREG1",
  "gene_name": "Protein CREG1",
  "term_id": "UNKNOWN:0001",
  "gene": "UniProtKB:O75629"
}